{
  "gene": "UniProtKB:P10632",
  "gene_symbol": "CYP2C8",
  "gene_name": "Cytochrome P450 2C8",
  "term_label": "xenobiotic catabolic process",
  "term_id": "GO:0042178"
}